glycolytic process from sucrose through glucose and fructose [GO:0061706] (biological process) Definition: The chemical reactions and pathways resulting in the breakdown of sucrose into pyruvate through both glucose and fructose intermediates, with the concomitant production of a small amount of ATP and the reduction of NAD(P) to NAD(P)H. Glycolysis begins with the metabolism of a carbohydrate to generate products that can enter the pathway and ends with the production of pyruvate. Pyruvate may be converted to acetyl-coenzyme A, ethanol, lactate, or other small molecules. References: PMID:15012287 Sources: GOC:dph, GOC:glycolysis, MetaCyc:PWY-1042 Relationships: is a type of glycolytic process through fructose-6-phosphate [GO:0061615]; is a type of glycolytic process from sucrose [GO:0061704]; has part GO:0061705